hexadecanol dehydrogenase (NAD+) activity [GO:0047978] (molecular function) Definition: Catalysis of the reaction: hexadecanol + NAD+ = hexadecanal + NADH. Also known as: hexadecanol dehydrogenase activity, hexadecanol:NAD+ oxidoreductase activity Relationships: is a type of alcohol dehydrogenase (NAD+) activity [GO:0004022] Sources: EC:1.1.1.164, MetaCyc:HEXADECANOL-DEHYDROGENASE-RXN